{
  "term_id": "GO:0005886",
  "gene_symbol": "BMPR1A",
  "gene": "UniProtKB:P36894",
  "term_label": "plasma membrane",
  "gene_name": "Bone morphogenetic protein receptor type-1A"
}